{
  "gene_symbol": "PNOC",
  "gene_name": "Prepronociceptin",
  "term_label": "axon terminus",
  "gene": "UniProtKB:Q13519",
  "term_id": "GO:0043679"
}